{
  "gene": "UniProtKB:P13747",
  "term_id": "GO:0005102",
  "gene_name": "HLA class I histocompatibility antigen, alpha chain E",
  "gene_symbol": "HLA-E",
  "term_label": "signaling receptor binding"
}